{
  "term_label": "muscle structure development",
  "gene_name": "PDZ and LIM domain protein 4",
  "gene": "UniProtKB:P50479",
  "gene_symbol": "PDLIM4",
  "term_id": "GO:0061061"
}